{
  "term_id": "GO:1905349",
  "gene_name": "Centrosomal protein of 290 kDa",
  "term_label": "ciliary transition zone assembly",
  "gene": "UniProtKB:O15078",
  "gene_symbol": "CEP290"
}